{
  "gene": "UniProtKB:P17030",
  "gene_name": "Zinc finger protein 25",
  "gene_symbol": "ZNF25",
  "term_id": "GO:0000981",
  "term_label": "DNA-binding transcription factor activity, RNA polymerase II-specific"
}